pectoral fin development [GO:0033339] (biological process) Sources: GOC:dgh Definition: The process whose specific outcome is the progression of the pectoral fin over time, from its formation to the mature structure. Relationships: is a type of fin development [GO:0033333]; is a type of limb development [GO:0060173]